{
  "gene": "UniProtKB:Q9Y6X6",
  "term_label": "myosin complex",
  "gene_name": "Unconventional myosin-XVI",
  "term_id": "GO:0016459",
  "gene_symbol": "MYO16"
}